response to hydroxyisoflavone [GO:0033594] (biological process) Definition: Any process that results in a change in state or activity of a cell or an organism (in terms of movement, secretion, enzyme production, gene expression, etc.) as a result of a hydroxyisoflavone stimulus. Sources: GOC:mah Subtypes: response to genistein [GO:0033595], cellular response to hydroxyisoflavone [GO:0071413] Relationships: is a type of response to phenylpropanoid [GO:0080184]; is a type of GO:1901654